{
  "term_label": "neuron projection extension",
  "gene_symbol": "NRN1",
  "term_id": "GO:1990138",
  "gene": "UniProtKB:Q9NPD7",
  "gene_name": "Neuritin"
}